{
  "term_id": "GO:0005096",
  "gene_name": "Ras GTPase-activating protein 3",
  "term_label": "GTPase activator activity",
  "gene_symbol": "RASA3",
  "gene": "UniProtKB:Q14644"
}